{
  "term_label": "Unknown cellular component",
  "gene_name": "Transmembrane O-methyltransferase",
  "term_id": "UNKNOWN:0003",
  "gene": "UniProtKB:Q8WZ04",
  "gene_symbol": "TOMT"
}